NADH dehydrogenase activity [GO:0003954] (molecular function) Sources: RHEA:11356 Relationships: is_a oxidoreductase activity, acting on NAD(P)H [GO:0016651] Definition: Catalysis of the reaction: NADH + H+ + acceptor = NAD+ + reduced acceptor. Subtypes: NADH dehydrogenase (quinone) (non-electrogenic) activity [GO:0050136] Also known as: diaphorase activity, NADH-menadione oxidoreductase activity, NADH:cytochrome c oxidoreductase activity, DPNH diaphorase activity, NADH diaphorase activity, NADH hydrogenase activity, NADH oxidoreductase activity, NADH2 dehydrogenase activity, NADH:(acceptor) oxidoreductase activity, NADH:acceptor oxidoreductase activity, beta-NADH dehydrogenase dinucleotide activity, cytochrome c reductase activity, dihydrocodehydrogenase I dehydrogenase activity, dihydronicotinamide adenine dinucleotide dehydrogenase activity, diphosphopyridine diaphorase activity, diphosphopyrinase activity, reduced diphosphopyridine nucleotide diaphorase activity, type 1 dehydrogenase activity, type I dehydrogenase activity